{
  "term_id": "GO:0015232",
  "gene_name": "Heme transporter FLVCR2",
  "gene": "UniProtKB:Q9UPI3",
  "term_label": "heme transmembrane transporter activity",
  "gene_symbol": "FLVCR2"
}